positive regulation of response to pullulan [GO:1900520] (biological process) Also known as: up regulation of response to pullulan, up-regulation of response to pullulan, upregulation of response to pullulan, activation of response to pullulan Relationships: is a type of positive regulation of response to stimulus [GO:0048584]; is a type of regulation of response to pullulan [GO:1900518]; positively regulates GO:0044592 Sources: GOC:TermGenie, GOC:mengo_curators Definition: Any process that activates or increases the frequency, rate or extent of response to pullulan.